positive regulation of mitotic cell cycle spindle assembly checkpoint [GO:0090267] (biological process) Definition: Any process that increases the rate, frequency, or extent of the mitotic cell cycle spindle assembly checkpoint, a cell cycle checkpoint that delays the metaphase/anaphase transition of a mitotic nuclear division until the spindle is correctly assembled and chromosomes are attached to the spindle. Relationships: is a type of positive regulation of cell cycle process [GO:0090068]; is a type of positive regulation of spindle checkpoint [GO:0090232]; is_a regulation of mitotic cell cycle spindle assembly checkpoint [GO:0090266]; positively regulates GO:0007094 Sources: GOC:mah, GOC:vw Subtypes: activation of mitotic cell cycle spindle assembly checkpoint [GO:0090268]